{
  "term_id": "UNKNOWN:0001",
  "gene_name": "Putative uncharacterized protein UNQ9165_PRO28630",
  "gene": "UniProtKB:Q6UXU0",
  "gene_symbol": "UNQ9165_PRO28630",
  "term_label": "Unknown molecular function"
}